{
  "term_id": "GO:0009952",
  "gene_name": "Transcription cofactor HES-6",
  "term_label": "anterior/posterior pattern specification",
  "gene": "UniProtKB:Q96HZ4",
  "gene_symbol": "HES6"
}